{
  "gene_symbol": "SMIM1",
  "term_label": "cell surface",
  "term_id": "GO:0009986",
  "gene": "UniProtKB:B2RUZ4",
  "gene_name": "Small integral membrane protein 1"
}